{
  "gene_name": "Coiled-coil domain-containing protein 124",
  "term_id": "GO:0006366",
  "term_label": "transcription by RNA polymerase II",
  "gene_symbol": "CCDC124",
  "gene": "UniProtKB:Q96CT7"
}